{
  "term_label": "Unknown biological process",
  "gene_name": "4-galactosyl-N-acetylglucosaminide 3-alpha-L-fucosyltransferase FUT6",
  "gene": "UniProtKB:P51993",
  "gene_symbol": "FUT6",
  "term_id": "UNKNOWN:0002"
}